{
  "gene_symbol": "CTSE",
  "gene": "UniProtKB:P14091",
  "gene_name": "Cathepsin E",
  "term_label": "antigen processing and presentation of exogenous peptide antigen via MHC class II",
  "term_id": "GO:0019886"
}